positive regulation of neuromuscular junction development [GO:1904398] (biological process) Also known as: positive regulation of neuromuscular junction organization, up regulation of neuromuscular junction development, up regulation of neuromuscular junction organization, up-regulation of neuromuscular junction development, up-regulation of neuromuscular junction organization, upregulation of neuromuscular junction development, upregulation of neuromuscular junction organization, activation of neuromuscular junction development, activation of neuromuscular junction organization, activation of NMJ stability, activation of neuromuscular junction stability, positive regulation of NMJ stability, positive regulation of neuromuscular junction stability, up regulation of NMJ stability, up regulation of neuromuscular junction stability, up-regulation of NMJ stability, up-regulation of neuromuscular junction stability, upregulation of NMJ stability, upregulation of neuromuscular junction stability Relationships: is a type of positive regulation of cellular component organization [GO:0051130]; is_a regulation of neuromuscular junction development [GO:1904396]; positively regulates neuromuscular junction development [GO:0007528] References: PMID:7722643 Sources: GOC:TermGenie, GO_REF:0000058 Subtypes: GO:0045887 Definition: Any process that activates or increases the frequency, rate or extent of neuromuscular junction development.